{
  "term_label": "presynaptic membrane",
  "gene_symbol": "UNC13C",
  "gene_name": "Protein unc-13 homolog C",
  "gene": "UniProtKB:Q8NB66",
  "term_id": "GO:0042734"
}